alphaV-beta3 integrin-NOV complex [GO:0071118] (CC) Definition: A protein complex that consists of an alphaV-beta3 integrin complex bound to the extracellular matrix protein NOV. References: PMID:12902636 Also known as: ITGAV-ITGB3-FN-1-NOV complex Relationships: is a type of plasma membrane protein complex [GO:0098797]